{
  "term_id": "GO:0030992",
  "gene_name": "TRAF3-interacting protein 1",
  "term_label": "intraciliary transport particle B",
  "gene_symbol": "TRAF3IP1",
  "gene": "UniProtKB:Q8TDR0"
}